hydrotropism [GO:0010274] (BP) Sources: ISBN:0395825172 Relationships: is a type of tropism [GO:0009606] Definition: Growth or movement in a sessile organism toward or away from water, as of the roots of a plant.